{
  "gene_name": "Ankyrin repeat domain-containing protein 23",
  "gene": "UniProtKB:Q86SG2",
  "term_id": "GO:0005634",
  "term_label": "nucleus",
  "gene_symbol": "ANKRD23"
}